{
  "gene_name": "GMP reductase 1",
  "gene": "UniProtKB:P36959",
  "term_id": "UNKNOWN:0001",
  "term_label": "Unknown molecular function",
  "gene_symbol": "GMPR"
}